CCR4-NOT core complex [GO:0030015] (cellular component) Definition: The core of the CCR4-NOT complex. In Saccharomyces the CCR4-NOT core complex comprises Ccr4p, Caf1p, Caf40p, Caf130p, Not1p, Not2p, Not3p, Not4p, and Not5p. References: PMID:11113136 Sources: GOC:sart Relationships: is a type of intracellular protein-containing complex [GO:0140535]; is part of CCR4-NOT complex [GO:0030014]